{
  "term_id": "GO:0030674",
  "gene_symbol": "SH3BGR",
  "gene": "UniProtKB:P55822",
  "term_label": "protein-macromolecule adaptor activity",
  "gene_name": "SH3 domain-binding glutamic acid-rich protein"
}